{
  "gene": "UniProtKB:P00390",
  "term_id": "GO:0004362",
  "gene_symbol": "GSR",
  "term_label": "glutathione-disulfide reductase (NADPH) activity",
  "gene_name": "Glutathione reductase, mitochondrial"
}